{
  "gene": "UniProtKB:Q7RTU0",
  "term_label": "DNA-binding transcription factor activity, RNA polymerase II-specific",
  "gene_symbol": "TCF24",
  "gene_name": "Transcription factor 24",
  "term_id": "GO:0000981"
}